{
  "gene_name": "3-phosphoinositide-dependent protein kinase 1",
  "gene_symbol": "PDPK1",
  "gene": "UniProtKB:O15530",
  "term_id": "GO:0035556",
  "term_label": "intracellular signal transduction"
}